{
  "gene_name": "Transcription factor RelB",
  "gene": "UniProtKB:Q01201",
  "gene_symbol": "RELB",
  "term_label": "RNA polymerase II cis-regulatory region sequence-specific DNA binding",
  "term_id": "GO:0000978"
}